{
  "term_label": "outward rectifier potassium channel activity",
  "gene_name": "Potassium channel subfamily T member 1",
  "gene_symbol": "KCNT1",
  "term_id": "GO:0015271",
  "gene": "UniProtKB:Q5JUK3"
}